{
  "gene_name": "D-aminoacyl-tRNA deacylase 2",
  "gene": "UniProtKB:Q96FN9",
  "gene_symbol": "DTD2",
  "term_label": "tRNA metabolic process",
  "term_id": "GO:0006399"
}